cellular response to endothelin [GO:1990859] (biological process) References: PMID:16365184 Definition: Any process that results in a change in state or activity of a cell (in terms of movement, secretion, enzyme production, gene expression, etc.) as a result of an endothelin stimulus. Endothelin is any of three secretory vasoconstrictive peptides (endothelin-1, -2, -3). Relationships: is_a GO:0071375; is_a GO:1990839